{
  "gene_name": "Melanoma-associated antigen B3",
  "gene_symbol": "MAGEB3",
  "term_id": "GO:0000122",
  "gene": "UniProtKB:O15480",
  "term_label": "negative regulation of transcription by RNA polymerase II"
}